{
  "term_id": "UNKNOWN:0001",
  "term_label": "Unknown molecular function",
  "gene_symbol": "EMP2",
  "gene": "UniProtKB:P54851",
  "gene_name": "Epithelial membrane protein 2"
}